{
  "term_id": "GO:0005886",
  "gene_name": "Epsin-2",
  "term_label": "plasma membrane",
  "gene": "UniProtKB:O95208",
  "gene_symbol": "EPN2"
}